{
  "gene_name": "Probable inactive peptidyl-prolyl cis-trans isomerase-like 6",
  "term_id": "UNKNOWN:0002",
  "gene_symbol": "PPIL6",
  "term_label": "Unknown biological process",
  "gene": "UniProtKB:Q8IXY8"
}